{
  "term_label": "heme biosynthetic process",
  "gene_name": "Delta-aminolevulinic acid dehydratase",
  "gene_symbol": "ALAD",
  "gene": "UniProtKB:P13716",
  "term_id": "GO:0006783"
}